peptidyl-aspartic acid phosphorylation [GO:0018217] (biological process) Sources: GOC:jl Subtypes: peptidyl-aspartic acid autophosphorylation [GO:1990938] Definition: The phosphorylation of peptidyl-aspartic acid. Relationships: is a type of protein phosphorylation [GO:0006468]; is a type of peptidyl-aspartic acid modification [GO:0018197]